phosphatidylinositol trisphosphate phosphatase activity [GO:0034594] (molecular function) Relationships: is a type of GO:0052866 Sources: GOC:mah Definition: Catalysis of the reaction: phosphatidylinositol trisphosphate + H2O = phosphatidylinositol bisphosphate + phosphate. Subtypes: phosphatidylinositol-3,4,5-trisphosphate 3-phosphatase activity [GO:0016314], phosphatidylinositol-3,4,5-trisphosphate 5-phosphatase activity [GO:0034485], phosphatidylinositol-1,4,5-trisphosphate 5-phosphatase activity [GO:0052867]